{
  "gene": "UniProtKB:P0DMR2",
  "term_label": "Unknown biological process",
  "gene_name": "Secretoglobin family 1C member 2",
  "gene_symbol": "SCGB1C2",
  "term_id": "UNKNOWN:0002"
}